{
  "term_id": "GO:0007099",
  "gene_name": "Centrosomal protein of 135 kDa",
  "term_label": "centriole replication",
  "gene": "UniProtKB:Q66GS9",
  "gene_symbol": "CEP135"
}